{
  "gene_name": "RAD50-interacting protein 1",
  "term_id": "UNKNOWN:0001",
  "term_label": "Unknown molecular function",
  "gene": "UniProtKB:Q6NUQ1",
  "gene_symbol": "RINT1"
}